{
  "gene": "UniProtKB:Q5T7M9",
  "term_id": "UNKNOWN:0001",
  "gene_name": "Divergent protein kinase domain 1A",
  "gene_symbol": "DIPK1A",
  "term_label": "Unknown molecular function"
}